{
  "gene_name": "Seizure protein 6 homolog",
  "term_id": "GO:0060074",
  "gene": "UniProtKB:Q53EL9",
  "gene_symbol": "SEZ6",
  "term_label": "synapse maturation"
}